RNA fragment catabolic process [GO:0000292] (biological process) Sources: GOC:mah Definition: The chemical reactions and pathways resulting in the breakdown of a fragment of RNA, such as excised introns or sequences removed from ribosomal RNA during processing. Relationships: is a type of GO:0006401 Also known as: RNA fragment breakdown, RNA fragment catabolism, RNA fragment degradation, group I intron catabolic process